{
  "term_id": "GO:0005085",
  "gene_name": "Translation initiation factor eIF-2B subunit beta",
  "gene_symbol": "EIF2B2",
  "term_label": "guanyl-nucleotide exchange factor activity",
  "gene": "UniProtKB:P49770"
}